{
  "term_label": "protein sumoylation",
  "term_id": "GO:0016925",
  "gene_name": "E3 SUMO-protein ligase NSE2",
  "gene_symbol": "NSMCE2",
  "gene": "UniProtKB:Q96MF7"
}